{
  "term_label": "chromatin",
  "gene": "UniProtKB:P62508",
  "gene_name": "Estrogen-related receptor gamma",
  "gene_symbol": "ESRRG",
  "term_id": "GO:0000785"
}